{
  "term_id": "GO:0005737",
  "gene_symbol": "DZIP1",
  "gene": "UniProtKB:Q86YF9",
  "term_label": "cytoplasm",
  "gene_name": "Cilium assembly protein DZIP1"
}